{
  "term_id": "UNKNOWN:0003",
  "term_label": "Unknown cellular component",
  "gene_symbol": "TRAJ49",
  "gene_name": "T cell receptor alpha joining 49 (Fragment)",
  "gene": "UniProtKB:A0A075B6Y0"
}